{
  "gene_symbol": "TRIM68",
  "gene": "UniProtKB:Q6AZZ1",
  "gene_name": "E3 ubiquitin-protein ligase TRIM68",
  "term_id": "GO:0010468",
  "term_label": "regulation of gene expression"
}